{
  "gene": "UniProtKB:Q9NZC2",
  "gene_symbol": "TREM2",
  "term_id": "GO:0060100",
  "term_label": "positive regulation of phagocytosis, engulfment",
  "gene_name": "Triggering receptor expressed on myeloid cells 2"
}